protein localization to horsetail-astral microtubule array [GO:1903696] (biological process) Also known as: protein localisation in horsetail-astral microtubule array, protein localisation to horsetail-astral microtubule array, protein localization in horsetail-astral microtubule array Relationships: is a type of protein localization to cortical microtubule cytoskeleton [GO:0072699] Definition: A process in which a protein is transported to, or maintained in, a location within a horsetail-astral microtubule array. References: PMID:11907273 Sources: GOC:TermGenie, GO_REF:0000087